{
  "gene": "UniProtKB:Q8TC56",
  "term_label": "Unknown biological process",
  "gene_symbol": "GARIN3",
  "term_id": "UNKNOWN:0002",
  "gene_name": "Golgi-associated RAB2 interactor protein 3"
}